{
  "gene": "UniProtKB:O15372",
  "term_id": "GO:0008237",
  "gene_name": "Eukaryotic translation initiation factor 3 subunit H",
  "term_label": "metallopeptidase activity",
  "gene_symbol": "EIF3H"
}